{
  "gene": "UniProtKB:Q92858",
  "term_id": "GO:0007423",
  "gene_symbol": "ATOH1",
  "gene_name": "Transcription factor ATOH1",
  "term_label": "sensory organ development"
}